{
  "term_id": "GO:0015277",
  "gene": "UniProtKB:P39086",
  "gene_symbol": "GRIK1",
  "gene_name": "Glutamate receptor ionotropic, kainate 1",
  "term_label": "kainate selective glutamate receptor activity"
}